{
  "gene": "UniProtKB:Q3SY46",
  "gene_name": "Keratin-associated protein 13-3",
  "term_label": "Unknown biological process",
  "gene_symbol": "KRTAP13-3",
  "term_id": "UNKNOWN:0002"
}